{
  "gene_symbol": "ARHGAP5",
  "gene": "UniProtKB:Q13017",
  "term_id": "GO:0007266",
  "gene_name": "Rho GTPase-activating protein 5",
  "term_label": "Rho protein signal transduction"
}